{
  "gene_symbol": "CDC42SE2",
  "gene": "UniProtKB:Q9NRR3",
  "term_label": "plasma membrane",
  "gene_name": "CDC42 small effector protein 2",
  "term_id": "GO:0005886"
}